{
  "gene_name": "Pre-mRNA 3'-end-processing factor FIP1",
  "term_label": "Unknown molecular function",
  "term_id": "UNKNOWN:0001",
  "gene_symbol": "FIP1L1",
  "gene": "UniProtKB:Q6UN15"
}